{
  "term_label": "intracellular signal transduction",
  "term_id": "GO:0035556",
  "gene_name": "Serine_threonine-protein kinase N2",
  "gene_symbol": "PKN2",
  "gene": "UniProtKB:Q16513"
}